phagolysosome assembly [GO:0001845] (biological process) Also known as: late phagosome biosynthesis, late phagosome formation, phagolysosome formation Relationships: is a type of lysosome organization [GO:0007040]; is a type of vesicle organization [GO:0016050]; is_a organelle assembly [GO:0070925]; is part of phagocytosis [GO:0006909]; is part of phagosome maturation [GO:0090382] Sources: GOC:add, ISBN:0781735149 Subtypes: phagolysosome assembly involved in apoptotic cell clearance [GO:0090387] Definition: The process that results in the fusion of a phagosome, a vesicle formed by phagocytosis, with a lysosome.